signal release from synapse [GO:0099643] (biological process) Definition: Any signal release from a synapse. Sources: GOC:dos Relationships: is a type of GO:0023061; is part of GO:0099536; occurs in synapse [GO:0045202] Subtypes: neurotransmitter secretion [GO:0007269], synaptic vesicle exocytosis [GO:0016079]